integrin activation [GO:0033622] (biological process) Regulation: regulated by GO:0033623; negatively regulated by negative regulation of integrin activation [GO:0033624]; positively regulated by positive regulation of integrin activation [GO:0033625] Relationships: is a type of protein-containing complex assembly [GO:0065003] Also known as: integrin complex activation, integrin complex assembly References: PMID:12213832, PMID:14754902 Sources: GOC:add Definition: The aggregation, arrangement and bonding together of an integrin, a heterodimeric adhesion receptor formed by the non-covalent association of particular alpha and beta subunits, that lead to the increased affinity of the integrin for its extracellular ligands.